{
  "gene_symbol": "ST8SIA6",
  "term_id": "GO:0003828",
  "gene_name": "Alpha-2,8-sialyltransferase 8F",
  "term_label": "alpha-N-acetylneuraminate alpha-2,8-sialyltransferase activity",
  "gene": "UniProtKB:P61647"
}